{
  "term_label": "proteasome-mediated ubiquitin-dependent protein catabolic process",
  "gene_symbol": "TRIP12",
  "gene_name": "E3 ubiquitin-protein ligase TRIP12",
  "term_id": "GO:0043161",
  "gene": "UniProtKB:Q14669"
}